{
  "term_id": "GO:0005886",
  "gene_name": "Talin-1",
  "gene_symbol": "TLN1",
  "term_label": "plasma membrane",
  "gene": "UniProtKB:Q9Y490"
}